pyridoxal phosphate binding [GO:0030170] (MF) Sources: GOC:mah, ISBN:0198506732 Definition: Binding to pyridoxal 5' phosphate, 3-hydroxy-5-(hydroxymethyl)-2-methyl4-pyridine carboxaldehyde 5' phosphate, the biologically active form of vitamin B6. Relationships: is_a GO:0043168; is a type of vitamin B6 binding [GO:0070279]